{
  "gene": "UniProtKB:Q12979",
  "gene_name": "Active breakpoint cluster region-related protein",
  "term_label": "Unknown biological process",
  "gene_symbol": "ABR",
  "term_id": "UNKNOWN:0002"
}